{
  "term_label": "voltage-gated potassium channel complex",
  "gene_symbol": "KCNC1",
  "term_id": "GO:0008076",
  "gene_name": "Potassium voltage-gated channel subfamily C member 1",
  "gene": "UniProtKB:P48547"
}